{
  "gene_name": "Testicular haploid expressed gene protein-like",
  "gene_symbol": "THEGL",
  "term_label": "Unknown molecular function",
  "gene": "UniProtKB:P0DJG4",
  "term_id": "UNKNOWN:0001"
}